regulation of polarized epithelial cell differentiation [GO:0030860] (biological process) Subtypes: negative regulation of polarized epithelial cell differentiation [GO:0030861], positive regulation of polarized epithelial cell differentiation [GO:0030862] Definition: Any process that modulates the frequency, rate or extent of polarized epithelial cell differentiation. Sources: GOC:mah Relationships: is a type of GO:0030856; is a type of GO:2000027; regulates polarized epithelial cell differentiation [GO:0030859]